{
  "gene_symbol": "PTPN22",
  "term_label": "regulation of non-canonical NF-kappaB signal transduction",
  "gene": "UniProtKB:Q9Y2R2",
  "gene_name": "Tyrosine-protein phosphatase non-receptor type 22",
  "term_id": "GO:1901222"
}